{
  "gene_symbol": "CATIP",
  "gene": "UniProtKB:Q7Z7H3",
  "term_id": "GO:0044782",
  "gene_name": "Ciliogenesis-associated TTC17-interacting protein",
  "term_label": "cilium organization"
}